{
  "gene_name": "TBC1 domain family member 30",
  "term_id": "UNKNOWN:0003",
  "gene": "UniProtKB:Q9Y2I9",
  "gene_symbol": "TBC1D30",
  "term_label": "Unknown cellular component"
}